positive regulation of optical nerve axon regeneration [GO:1905593] (biological process) Definition: Any process that activates or increases the frequency, rate or extent of optical nerve axon regeneration. Relationships: is a type of positive regulation of axon regeneration [GO:0048680]; is a type of regulation of optical nerve axon regeneration [GO:1905591]; positively regulates optical nerve axon regeneration [GO:0101027] Also known as: up regulation of optical nerve axon regeneration, up-regulation of optical nerve axon regeneration, upregulation of optical nerve axon regeneration, activation of optical nerve axon regeneration References: PMID:16699509 Sources: GOC:TermGenie, GO_REF:0000058